dihydroorotate dehydrogenase (NADP+) activity [GO:0050158] (MF) Also known as: orotate reductase (NADPH) activity, (S)-dihydroorotate:NADP+ oxidoreductase activity, L-5,6-dihydro-orotate:NAD oxidoreductase activity, dihydro-orotic dehydrogenase activity, orotate reductase activity Definition: Catalysis of the reaction: (S)-dihydroorotate + NADP+ = H+ + NADPH + orotate. Sources: RHEA:14861 Relationships: is a type of dihydroorotate dehydrogenase activity [GO:0004152]; is a type of oxidoreductase activity, acting on the CH-CH group of donors, NAD or NADP as acceptor [GO:0016628]